{
  "gene_symbol": "CHMP7",
  "gene_name": "Charged multivesicular body protein 7",
  "gene": "UniProtKB:Q8WUX9",
  "term_label": "Unknown molecular function",
  "term_id": "UNKNOWN:0001"
}